{
  "gene_name": "E3 ubiquitin-protein ligase CBL-C",
  "term_id": "GO:0030971",
  "term_label": "receptor tyrosine kinase binding",
  "gene_symbol": "CBLC",
  "gene": "UniProtKB:Q9ULV8"
}